{
  "term_label": "cytosol",
  "gene_name": "S100P-binding protein",
  "term_id": "GO:0005829",
  "gene": "UniProtKB:Q96BU1",
  "gene_symbol": "S100PBP"
}